ethylene-activated signaling pathway [GO:0009873] (biological process) References: PMID:24012247 Sources: GOC:jy Also known as: ethene mediated signalling pathway, ethene mediated signaling pathway, ethylene mediated signaling pathway, ethylene mediated signalling pathway, ethylene signal transduction, ethylene signaling pathway Subtypes: GO:0009866, jasmonic acid and ethylene-dependent systemic resistance, ethylene mediated signaling pathway [GO:0009871] Definition: The series of molecular signals generated by the reception of ethylene (ethene, C2H4) by a receptor and ending with modulation of a cellular process, e.g. transcription. Relationships: is_a phosphorelay signal transduction system [GO:0000160]; is a type of hormone-mediated signaling pathway [GO:0009755]; BFO_0000050 cellular response to ethylene stimulus [GO:0071369] Regulation: regulated by GO:0010104; negatively regulated by negative regulation of ethylene-activated signaling pathway [GO:0010105]